trans-Golgi-derived vesicle fusion with Golgi medial cisterna membrane [GO:1990692] (biological process) Also known as: trans-Golgi-derived vesicle fusion with medial-Golgi cisterna membrane Relationships: is a type of Golgi vesicle fusion to target membrane [GO:0048210]; is a type of GO:0048280; is part of retrograde transport, vesicle recycling within Golgi [GO:0000301] References: PMID:16038056, PMID:24119662 Sources: GOC:bhm Definition: The joining of the lipid bilayer membrane around a trans-Golgi-derived vesicle to the lipid bilayer membrane around the medial-Golgi cisterna. Such vesicles include COPI-coated transport vesicles involved in retrograde transport.